{
  "gene": "UniProtKB:Q8NDN9",
  "term_id": "UNKNOWN:0002",
  "term_label": "Unknown biological process",
  "gene_symbol": "RCBTB1",
  "gene_name": "RCC1 and BTB domain-containing protein 1"
}